{
  "term_id": "GO:0014069",
  "gene": "UniProtKB:P24588",
  "term_label": "postsynaptic density",
  "gene_symbol": "AKAP5",
  "gene_name": "A-kinase anchor protein 5"
}